{
  "gene_name": "Agouti-related protein",
  "gene": "UniProtKB:O00253",
  "term_label": "neuropeptide hormone activity",
  "gene_symbol": "AGRP",
  "term_id": "GO:0005184"
}